positive regulation of eclosion [GO:0045805] (biological process) Definition: Any process that activates or increases the frequency, rate or extent of eclosion. Also known as: up regulation of eclosion, up-regulation of eclosion, upregulation of eclosion, activation of eclosion, stimulation of eclosion Sources: GOC:go_curators Relationships: is a type of GO:0007563; is a type of positive regulation of multicellular organismal process [GO:0051240]; positively regulates GO:0007562